discadenine catabolic process [GO:0034269] (biological process) Definition: The chemical reactions and pathways resulting in the breakdown of discadenine, (2S)-2-amino-4-{6-[(3-methylbut-2-en-1-yl)amino]-3H-purin-3-yl}butanoic acid. Relationships: is a type of cytokinin catabolic process [GO:0009823]; is a type of GO:0072523; is a type of GO:0170035; is a type of non-proteinogenic amino acid catabolic process [GO:0170044] Also known as: discadenine breakdown, discadenine catabolism, discadenine degradation Sources: GOC:mah